{
  "gene_symbol": "TESC",
  "term_id": "GO:0005886",
  "gene_name": "Calcineurin B homologous protein 3",
  "gene": "UniProtKB:Q96BS2",
  "term_label": "plasma membrane"
}